sucrose catabolic process to fructose-6-phosphate through glucose and fructose [GO:0061705] (biological process) References: PMID:15012287 Sources: GOC:dph, GOC:glycolysis, MetaCyc:PWY-621 Relationships: is a type of sucrose catabolic process [GO:0005987]; has part glucokinase activity [GO:0004340]; has part GO:0004347; has part sucrose alpha-glucosidase activity [GO:0004575]; has part fructokinase activity [GO:0008865] Definition: The chemical reactions and pathways resulting in the breakdown of sucrose, to yield fructose-6-phosphate through both glucose and fructose intermediates.